 [oboInOwl#status]